{
  "term_id": "GO:0035493",
  "term_label": "SNARE complex assembly",
  "gene_name": "Vesicle-associated membrane protein 3",
  "gene_symbol": "VAMP3",
  "gene": "UniProtKB:Q15836"
}